{
  "gene_symbol": "STRN3",
  "term_id": "GO:0090443",
  "gene": "UniProtKB:Q13033",
  "term_label": "FAR/SIN/STRIPAK complex",
  "gene_name": "Striatin-3"
}